vertebrate eye-specific patterning [GO:0150064] (BP) Relationships: is a type of regionalization [GO:0003002]; is part of central nervous system development [GO:0007417]; is part of visual system development [GO:0150063] Also known as: eye-specific patterning, eye-specific segregation, vertebrate eye-specific segregation, binocular vision development Definition: Early postnatal vertebrate developmental process, during which axons of retinal ganglion cells (RGCs), transmitting overlapping inputs from both eyes, segregate into distinct eye-specific non-overlapping regions in the dorsal lateral geniculate nucleus (dLGN) of the thalamus. References: PMID:16025107, PMID:22632727, PMID:29322522 Sources: GOC:aruk, GOC:bc